{
  "gene_name": "Prostate androgen-regulated mucin-like protein 1",
  "gene": "UniProtKB:Q6UWI2",
  "gene_symbol": "PARM1",
  "term_id": "GO:0005770",
  "term_label": "late endosome"
}